baroreceptor response to decreased systemic arterial blood pressure [GO:0001982] (biological process) Relationships: is a type of regulation of systemic arterial blood pressure by carotid sinus baroreceptor feedback [GO:0001978]; is a type of GO:0003084 Definition: The lowering of the number of nerve impulses from baroreceptors as a result of decreased stretch of an artery that results in an increased in sympathetic nerve impulses to peripheral blood vessels. Sources: GOC:dph, GOC:mtg_cardio, ISBN:0323031951, ISBN:0721643949